indole-3-acetate beta-glucosyltransferase activity [GO:0047215] (molecular function) Definition: Catalysis of the reaction: (indol-3-yl)acetate + UDP-D-glucose = 1-O-(indol-3-ylacetyl)-beta-D-glucose + UDP. Relationships: is a type of GO:0035251 Sources: EC:2.4.1.121, RHEA:14921 Also known as: UDP-glucose:auxin glucosyltransferase activity, UDP-glucose:indol-3-acetic acid glucosyltransferase activity, IAA-Glu synthetase activity, IAA-glucose synthase activity, IAGlu synthase activity, UDP-glucose:(indol-3-yl)acetate beta-D-glucosyltransferase activity, UDP-glucose:indol-3-ylacetate glucosyl-transferase activity, UDP-glucose:indol-3-ylacetate glucosyltransferase activity, UDPG-indol-3-ylacetyl glucosyl transferase activity, UDPglucose:indole-3-acetate beta-D-glucosyltransferase activity, indol-3-ylacetylglucose synthase activity, uridine diphosphoglucose-indoleacetate glucosyltransferase activity